{
  "gene": "UniProtKB:A8MWK0",
  "gene_symbol": "FADS2B",
  "term_label": "lipid metabolic process",
  "term_id": "GO:0006629",
  "gene_name": "Putative fatty acid desaturase 2-like protein FADS2B"
}